{
  "term_id": "UNKNOWN:0002",
  "gene_symbol": "KRTAP21-2",
  "gene": "UniProtKB:Q3LI59",
  "gene_name": "Keratin-associated protein 21-2",
  "term_label": "Unknown biological process"
}